{
  "gene_name": "HEPACAM family member 2",
  "gene_symbol": "HEPACAM2",
  "term_label": "centrosome",
  "gene": "UniProtKB:A8MVW5",
  "term_id": "GO:0005813"
}